{
  "gene": "UniProtKB:O94886",
  "gene_name": "CSC1-like protein 1",
  "gene_symbol": "TMEM63A",
  "term_id": "UNKNOWN:0002",
  "term_label": "Unknown biological process"
}